{
  "gene_name": "CMP-N-acetylneuraminate-beta-1,4-galactoside alpha-2,3-sialyltransferase",
  "term_id": "UNKNOWN:0002",
  "gene": "UniProtKB:Q11203",
  "gene_symbol": "ST3GAL3",
  "term_label": "Unknown biological process"
}